{
  "term_label": "defense response to Gram-negative bacterium",
  "gene_name": "Bactericidal permeability-increasing protein",
  "gene": "UniProtKB:P17213",
  "term_id": "GO:0050829",
  "gene_symbol": "BPI"
}